monoacylglycerol metabolic process [GO:0046462] (biological process) Relationships: is a type of acylglycerol metabolic process [GO:0006639] Sources: ISBN:0198506732 Also known as: monoacylglycerol metabolism, monoglyceride metabolic process, monoglyceride metabolism Subtypes: monoacylglycerol biosynthetic process [GO:0006640], monoacylglycerol catabolic process [GO:0052651] Definition: The chemical reactions and pathways involving monoacylglycerol, any ester of glycerol in which any one of its hydroxyl groups has been acylated with a fatty acid, the other being non-esterified.